{
  "term_id": "GO:0004867",
  "gene_symbol": "SERPINA4",
  "gene": "UniProtKB:P29622",
  "gene_name": "Kallistatin",
  "term_label": "serine-type endopeptidase inhibitor activity"
}